{
  "gene_symbol": "LSM10",
  "term_id": "GO:0071209",
  "gene": "UniProtKB:Q969L4",
  "term_label": "U7 snRNA binding",
  "gene_name": "U7 snRNA-associated Sm-like protein LSm10"
}